{
  "term_label": "Unknown cellular component",
  "term_id": "UNKNOWN:0003",
  "gene": "UniProtKB:Q8N4F0",
  "gene_symbol": "BPIFB2",
  "gene_name": "BPI fold-containing family B member 2"
}